telomeric repeat-containing RNA transcription [GO:0097393] (biological process) Relationships: is_a DNA-templated transcription [GO:0006351] Also known as: TERRA transcription References: PMID:22139915 Sources: GOC:al Definition: The synthesis of telomeric repeat-containing RNA from a DNA template. A telomere is a complex of DNA and proteins that seals the end of a chromosome.